{
  "gene_symbol": "EDN3",
  "term_id": "GO:0005615",
  "gene": "UniProtKB:P14138",
  "gene_name": "Endothelin-3",
  "term_label": "extracellular space"
}